{
  "gene": "UniProtKB:Q8TF17",
  "term_label": "regulation of intracellular protein transport",
  "gene_symbol": "SH3TC2",
  "gene_name": "SH3 domain and tetratricopeptide repeat-containing protein 2",
  "term_id": "GO:0033157"
}